metanephric nephron tubule development [GO:0072234] (biological process) Subtypes: metanephric ascending thin limb development [GO:0072218], metanephric distal convoluted tubule development [GO:0072221], metanephric proximal convoluted tubule development [GO:0072229], metanephric proximal straight tubule development [GO:0072230], metanephric thick ascending limb development [GO:0072233], GO:0072235, metanephric loop of Henle development [GO:0072236], metanephric proximal tubule development [GO:0072237], metanephric connecting tubule development [GO:0072286] Sources: GOC:mtg_kidney_jan10 Definition: The progression of a metanephric nephron tubule over time, from its initial formation to the mature structure. A metanephric nephron tubule is an epithelial tube that is part of the metanephric nephron, the functional part of the metanephros. Relationships: is a type of nephron tubule development [GO:0072080]; is a type of GO:0072170; is a type of GO:0072243